{
  "term_label": "perinuclear region of cytoplasm",
  "gene": "UniProtKB:Q96LK8",
  "gene_name": "Spermatogenesis-associated protein 32",
  "gene_symbol": "SPATA32",
  "term_id": "GO:0048471"
}